{
  "gene": "UniProtKB:Q9UNM6",
  "term_id": "GO:0005634",
  "term_label": "nucleus",
  "gene_name": "26S proteasome non-ATPase regulatory subunit 13",
  "gene_symbol": "PSMD13"
}